regulation of ruffle assembly [GO:1900027] (biological process) Relationships: is a type of GO:0120032; regulates GO:0097178 Subtypes: negative regulation of ruffle assembly [GO:1900028], GO:1900029 Sources: GOC:TermGenie, GOC:yaf Definition: Any process that modulates the frequency, rate or extent of ruffle assembly. Also known as: regulation of membrane ruffle formation, regulation of membrane ruffling